geraniol dehydrogenase activity [GO:0047924] (molecular function) Also known as: geraniol:NADP+ oxidoreductase activity Relationships: is a type of GO:0016616 Definition: Catalysis of the reaction: geraniol + NADP+ = geranial + NADPH. Sources: EC:1.1.1.183, MetaCyc:GERANIOL-DEHYDROGENASE-RXN